{
  "term_id": "GO:0005634",
  "gene_symbol": "FAF1",
  "term_label": "nucleus",
  "gene": "UniProtKB:Q9UNN5",
  "gene_name": "FAS-associated factor 1"
}